{
  "term_label": "ATP hydrolysis activity",
  "gene": "UniProtKB:Q96Q89",
  "gene_symbol": "KIF20B",
  "gene_name": "Kinesin-like protein KIF20B",
  "term_id": "GO:0016887"
}